{
  "gene_symbol": "PPP3CA",
  "gene": "UniProtKB:Q08209",
  "term_label": "cytosol",
  "gene_name": "Protein phosphatase 3 catalytic subunit alpha",
  "term_id": "GO:0005829"
}